{
  "term_label": "respiratory chain complex IV",
  "term_id": "GO:0045277",
  "gene_name": "Cytochrome c oxidase subunit 4 isoform 2, mitochondrial",
  "gene_symbol": "COX4I2",
  "gene": "UniProtKB:Q96KJ9"
}